response to singlet oxygen [GO:0000304] (biological process) Sources: GOC:krc, ISBN:0124325653, ISBN:0198506732 Relationships: is a type of response to reactive oxygen species [GO:0000302] Definition: Any process that results in a change in state or activity of a cell or an organism (in terms of movement, secretion, enzyme production, gene expression, etc.) as a result of a singlet oxygen stimulus. Singlet oxygen is a dioxygen (O2) molecule in which two 2p electrons have similar spin. Singlet oxygen is more highly reactive than the form in which these electrons are of opposite spin, and it is produced in mutant chloroplasts lacking carotenoids and by leukocytes during metabolic burst. Subtypes: GO:0071452